{
  "gene_name": "Probable N-acetyltransferase 14",
  "gene_symbol": "NAT14",
  "term_label": "Unknown cellular component",
  "gene": "UniProtKB:Q8WUY8",
  "term_id": "UNKNOWN:0003"
}